{
  "gene_symbol": "GZMH",
  "term_label": "protein maturation",
  "gene": "UniProtKB:P20718",
  "gene_name": "Granzyme H",
  "term_id": "GO:0051604"
}